clathrin-sculpted monoamine transport vesicle [GO:0070081] (CC) Definition: A clathrin-sculpted lipid bilayer membrane-enclosed vesicle after clathrin release and containing monoamines. Sources: GOC:mg2 Relationships: is a type of transport vesicle [GO:0030133]; is a type of GO:0060198 Also known as: clathrin sculpted monoamine constitutive secretory pathway transport vesicle, clathrin sculpted monoamine transport vesicle